{
  "gene": "UniProtKB:Q86UR5",
  "gene_name": "Regulating synaptic membrane exocytosis protein 1",
  "term_id": "GO:0016082",
  "term_label": "synaptic vesicle priming",
  "gene_symbol": "RIMS1"
}